negative regulation of thyroid gland epithelial cell proliferation [GO:1904442] (biological process) References: PMID:17646383 Sources: GOC:TermGenie, GO_REF:0000058 Also known as: down regulation of thyroid gland epithelial cell proliferation, down-regulation of thyroid gland epithelial cell proliferation, downregulation of thyroid gland epithelial cell proliferation, down regulation of Hurthle cell proliferation, down regulation of thyroid follicular cell proliferation, down-regulation of Hurthle cell proliferation, down-regulation of thyroid follicular cell proliferation, downregulation of Hurthle cell proliferation, downregulation of thyroid follicular cell proliferation, inhibition of Hurthle cell proliferation, inhibition of thyroid follicular cell proliferation, inhibition of thyroid gland epithelial cell proliferation, negative regulation of Hurthle cell proliferation, negative regulation of thyroid follicular cell proliferation Definition: Any process that stops, prevents or reduces the frequency, rate or extent of thyroid gland epithelial cell proliferation. Relationships: is a type of negative regulation of epithelial cell proliferation [GO:0050680]; is a type of negative regulation of developmental process [GO:0051093]; is a type of negative regulation of multicellular organismal process [GO:0051241]; is a type of GO:1904441; negatively regulates thyroid gland epithelial cell proliferation [GO:1990789]